4'-methoxyisoflavone 2'-hydroxylase activity [GO:0047957] (molecular function) Definition: Catalysis of the reaction: formononetin + NADPH + O2 = 2'-hydroxyformononetin + NADP+ + H2O. Also known as: isoflavone 2'-monooxygenase activity, formononetin,NADPH:oxygen oxidoreductase (2'-hydroxylating) Relationships: is a type of GO:0016709 Sources: EC:1.14.14.89, MetaCyc:ISOFLAVONE-2-HYDROXYLASE-RXN